{
  "term_id": "GO:0035249",
  "gene_symbol": "GRID2",
  "gene": "UniProtKB:O43424",
  "term_label": "synaptic transmission, glutamatergic",
  "gene_name": "Glutamate receptor ionotropic, delta-2"
}